eukaryotic initiation factor eIF2 binding [GO:0071074] (molecular function) Relationships: is a type of translation initiation factor binding [GO:0031369] Definition: Binding to eukaryotic initiation factor eIF2, a protein complex involved in the initiation of ribosome-mediated translation. Sources: GOC:hjd